lombricine kinase activity [GO:0050059] (molecular function) Definition: Catalysis of the reaction: ATP + lombricine = ADP + N-phospholombricine. Also known as: ATP:lombricine N-phosphotransferase activity Relationships: is a type of kinase activity [GO:0016301]; is a type of GO:0016775 Sources: EC:2.7.3.5, MetaCyc:LOMBRICINE-KINASE-RXN